{
  "gene_symbol": "ACSL5",
  "term_label": "positive regulation of long-chain fatty acid import across plasma membrane",
  "term_id": "GO:0010747",
  "gene": "UniProtKB:Q9ULC5",
  "gene_name": "Long-chain-fatty-acid--CoA ligase 5"
}